plastoglobule organization [GO:0080177] (biological process) Relationships: is a type of GO:0016043; is part of chloroplast organization [GO:0009658] Definition: A process that is carried out at the cellular level which results in the assembly, arrangement of constituent parts, or disassembly of the plastoglobule. Plastoglobule is a lipoprotein particle present in chloroplasts. They are rich in non-polar lipids (triglycerides, esters) as well as in prenylquinones, plastoquinone and tocopherols. Plastoglobules are often associated with thylakoid membranes, suggesting an exchange of lipids with thylakoids. References: PMID:20813909 Also known as: plastoglobule organisation